{
  "term_id": "GO:0005634",
  "gene_symbol": "MT1L",
  "gene_name": "Metallothionein-1L",
  "term_label": "nucleus",
  "gene": "UniProtKB:Q93083"
}